regulation of lymphocyte chemotaxis [GO:1901623] (biological process) Relationships: is a type of regulation of leukocyte chemotaxis [GO:0002688]; is_a regulation of lymphocyte migration [GO:2000401]; regulates lymphocyte chemotaxis [GO:0048247] Subtypes: regulation of T cell chemotaxis [GO:0010819], positive regulation of lymphocyte chemotaxis [GO:0140131], negative regulation of lymphocyte chemotaxis [GO:1901624], regulation of natural killer cell chemotaxis [GO:2000501], regulation of B cell chemotaxis [GO:2000537] Definition: Any process that modulates the frequency, rate or extent of lymphocyte chemotaxis. Sources: GOC:TermGenie